mannosyl-glycoprotein endo-beta-N-acetylglucosaminidase activity [GO:0033925] (molecular function) Relationships: is a type of GO:0004553 Definition: Catalysis of the endohydrolysis of the N,N'-diacetylchitobiosyl unit in high-mannose glycopeptides and glycoproteins containing the -[Man(GlcNAc)2]Asn-structure. One N-acetyl-D-glucosamine residue remains attached to the protein; the rest of the oligosaccharide is released intact. Also known as: N,N'-diacetylchitobiosyl beta-N-acetylglucosaminidase activity, di-N-acetylchitobiosyl beta-N-acetylglucosaminidase activity, endo-N-acetyl-beta-D-glucosaminidase activity, endo-N-acetyl-beta-glucosaminidase activity, endo-beta-(1->4)-N-acetylglucosaminidase activity, endo-beta-N-acetylglucosaminidase D activity, endo-beta-N-acetylglucosaminidase F activity, endo-beta-N-acetylglucosaminidase H activity, endo-beta-N-acetylglucosaminidase L activity, endo-beta-N-acetylglucosaminidase activity, endo-beta-acetylglucosaminidase activity, endoglycosidase H activity, endoglycosidase S activity, glycopeptide-D-mannosyl-4-N-(N-acetyl-D-glucosaminyl)2-asparagine 1,4-N-acetyl-beta-glucosaminohydrolase activity, glycopeptide-D-mannosyl-N4-(N-acetyl-D-glucosaminyl)2-asparagine 1,4-N-acetyl-beta-glucosaminohydrolase activity, mannosyl-glycoprotein 1,4-N-acetamidodeoxy-beta-D-glycohydrolase activity, mannosyl-glycoprotein endo-beta-N-acetylglucosamidase activity Sources: EC:3.2.1.96